{
  "term_label": "centriole",
  "gene_symbol": "CEP76",
  "gene_name": "Centrosomal protein of 76 kDa",
  "gene": "UniProtKB:Q8TAP6",
  "term_id": "GO:0005814"
}